{
  "term_id": "GO:1990404",
  "gene_symbol": "PARP12",
  "term_label": "NAD+-protein mono-ADP-ribosyltransferase activity",
  "gene_name": "Protein mono-ADP-ribosyltransferase PARP12",
  "gene": "UniProtKB:Q9H0J9"
}